erythrulose reductase activity [GO:0047880] (molecular function) Also known as: D-erythrulose reductase activity, erythritol:NADP+ oxidoreductase activity Relationships: is a type of oxidoreductase activity, acting on the CH-OH group of donors, NAD or NADP as acceptor [GO:0016616] Sources: EC:1.1.1.162, RHEA:18005 Definition: Catalysis of the reaction: D-threitol + NADP+ = D-erythrulose + H+ + NADPH.